{
  "gene": "UniProtKB:P42684",
  "gene_name": "Tyrosine-protein kinase ABL2",
  "term_label": "protein tyrosine kinase activity",
  "term_id": "GO:0004713",
  "gene_symbol": "ABL2"
}